ventral disc crossbridge [GO:0097595] (cellular component) Definition: Structure horizontally linking adjacent microribbons of the ventral disc in Giardia species (trophozoite stage). The composition of crossbridges is not fully known yet. Relationships: is a type of cellular anatomical structure [GO:0110165]; is part of ventral disc [GO:0097597] Also known as: crossbridge, ventral disk crossbridge Sources: GOC:giardia Note: Due to the asymmetric nature of the Giardia trophozoite, this term is defined spatially as the trophozoite is viewed from the dorsal side, with the two nuclei dorsal to the ventral disc, and the ventral disc toward the anterior.